cellular response to cation stress [GO:0071473] (biological process) Relationships: is a type of response to cation stress [GO:0043157]; is a type of cellular response to salt stress [GO:0071472] Sources: GOC:mah Definition: Any process that results in a change in state or activity of a cell (in terms of movement, secretion, enzyme production, gene expression, etc.) as a result of cation stress, an increase or decrease in the concentration of positively charged ions in the environment.